{
  "term_label": "syncytium formation by plasma membrane fusion",
  "gene_symbol": "ERVFRD-1",
  "gene": "UniProtKB:P60508",
  "gene_name": "Syncytin-2",
  "term_id": "GO:0000768"
}